{
  "gene_symbol": "XKRY",
  "term_id": "UNKNOWN:0001",
  "gene": "UniProtKB:O14609",
  "term_label": "Unknown molecular function",
  "gene_name": "Testis-specific XK-related protein, Y-linked"
}